{
  "gene_name": "Phosphomannomutase 2",
  "gene_symbol": "PMM2",
  "term_id": "GO:0005829",
  "gene": "UniProtKB:O15305",
  "term_label": "cytosol"
}